host intracellular part [GO:0033646] (cellular component) Note: Note that this term is in the subset of terms that should not be used for direct gene product annotation. Instead, select a child term or, if no appropriate child term exists, please request a new term. Direct annotations to this term may be amended during annotation QC. Relationships: is a type of GO:0033643; is part of GO:0043656 Definition: Any constituent part of the living contents of a host cell; the matter contained within (but not including) the plasma membrane, usually taken to exclude large vacuoles and masses of secretory or ingested material. In eukaryotes it includes the nucleus and cytoplasm. The host is defined as the larger of the organisms involved in a symbiotic interaction. Subtypes: host cell cytoplasm [GO:0030430], host intracellular organelle [GO:0033647], host cell cytoplasm part [GO:0033655], host cell viral nucleoid [GO:0039643], host cell nuclear part [GO:0044094] Sources: GOC:pamgo_curators Also known as: host cell intracellular part